negative regulation of maltohexaose transport [GO:1900313] (biological process) Sources: GOC:TermGenie, GOC:mengo_curators Relationships: is a type of GO:1900298; is a type of regulation of maltohexaose transport [GO:1900312]; negatively regulates maltohexaose transport [GO:2001103] Also known as: down regulation of maltohexaose transport, down-regulation of maltohexaose transport, downregulation of maltohexaose transport, inhibition of maltohexaose transport Definition: Any process that stops, prevents or reduces the frequency, rate or extent of maltohexaose transport.